{
  "gene": "UniProtKB:P01768",
  "term_label": "antigen binding",
  "gene_symbol": "IGHV3-30",
  "term_id": "GO:0003823",
  "gene_name": "Immunoglobulin heavy variable 3-30"
}